{
  "gene_name": "Down syndrome critical region protein 4",
  "term_id": "UNKNOWN:0002",
  "term_label": "Unknown biological process",
  "gene_symbol": "DSCR4",
  "gene": "UniProtKB:P56555"
}